alanine-oxomalonate transaminase activity [GO:0047308] (molecular function) Relationships: is a type of transaminase activity [GO:0008483] Definition: Catalysis of the reaction: L-alanine + oxomalonate = aminomalonate + pyruvate. Sources: EC:2.6.1.47, RHEA:18809 Also known as: alanine-oxomalonate aminotransferase activity, L-alanine-ketomalonate transaminase activity, L-alanine:oxomalonate aminotransferase activity, alanine--oxomalonate aminotransferase activity, alanine-ketomalonate (mesoxalate) transaminase activity